{
  "term_label": "transmembrane receptor protein tyrosine kinase activity",
  "gene_name": "Leukocyte tyrosine kinase receptor",
  "gene": "UniProtKB:P29376",
  "term_id": "GO:0004714",
  "gene_symbol": "LTK"
}